{
  "term_label": "olfactory receptor activity",
  "gene_symbol": "OR2T35",
  "term_id": "GO:0004984",
  "gene_name": "Olfactory receptor 2T35",
  "gene": "UniProtKB:Q8NGX2"
}